regulation of glyoxylate cycle [GO:2000874] (biological process) Subtypes: negative regulation of glyoxylate cycle [GO:2000875], GO:2000876 Also known as: regulation of glyoxylate bypass Sources: GOC:dgf Definition: Any process that modulates the frequency, rate or extent of glyoxylate cycle. Relationships: is a type of GO:0006109; is a type of regulation of ketone metabolic process [GO:0010565]; is a type of regulation of small molecule metabolic process [GO:0062012]; regulates GO:0006097